{
  "gene": "UniProtKB:Q9Y6A5",
  "gene_symbol": "TACC3",
  "term_label": "centrosome",
  "gene_name": "Transforming acidic coiled-coil-containing protein 3",
  "term_id": "GO:0005813"
}